{
  "gene_symbol": "TEX26",
  "gene_name": "Testis-expressed protein 26",
  "term_label": "cytoplasm",
  "term_id": "GO:0005737",
  "gene": "UniProtKB:Q8N6G2"
}